{
  "term_label": "multi-eIF complex",
  "gene": "UniProtKB:Q14152",
  "gene_symbol": "EIF3A",
  "term_id": "GO:0043614",
  "gene_name": "Eukaryotic translation initiation factor 3 subunit A"
}